positive regulation of [2Fe-2S] cluster assembly [GO:1900489] (biological process) Also known as: positive regulation of 2Fe-2S cluster assembly, up regulation of 2Fe-2S cluster assembly, up regulation of [2Fe-2S] cluster assembly, up-regulation of 2Fe-2S cluster assembly, up-regulation of [2Fe-2S] cluster assembly, upregulation of 2Fe-2S cluster assembly, upregulation of [2Fe-2S] cluster assembly, activation of 2Fe-2S cluster assembly, activation of [2Fe-2S] cluster assembly, activation of [2Fe-2S] cluster biosynthetic process, positive regulation of [2Fe-2S] cluster biosynthetic process, up regulation of [2Fe-2S] cluster biosynthetic process, up-regulation of [2Fe-2S] cluster biosynthetic process, upregulation of [2Fe-2S] cluster biosynthetic process Relationships: is a type of GO:1900487; is a type of positive regulation of iron-sulfur cluster assembly [GO:1903331]; RO_0002213 [2Fe-2S] cluster assembly [GO:0044571] Definition: Any process that activates or increases the frequency, rate or extent of [2Fe-2S] cluster assembly. Sources: GOC:TermGenie, GOC:mengo_curators, GOC:pr